{
  "gene": "UniProtKB:Q8IYU2",
  "term_label": "nucleus",
  "gene_symbol": "HACE1",
  "gene_name": "E3 ubiquitin-protein ligase HACE1",
  "term_id": "GO:0005634"
}